{
  "gene": "UniProtKB:Q8IU68",
  "gene_name": "Transmembrane channel-like protein 8",
  "term_id": "UNKNOWN:0002",
  "term_label": "Unknown biological process",
  "gene_symbol": "TMC8"
}